collagen type XXVII trimer [GO:1990325] (cellular component) Definition: A collagen homotrimer of alpha1(XXVII) chains. These trimers form thin, non-striated fibrils. Type XXVII collagen triple helices play a role during the calcification of cartilage and the transition of cartilage to bone. References: PMID:17876790, PMID:21421911 Relationships: is a type of fibrillar collagen trimer [GO:0005583]